negative regulation of transcytosis [GO:1904299] (BP) References: PMID:9664076 Sources: GOC:TermGenie, GO_REF:0000058 Relationships: is a type of negative regulation of cellular process [GO:0048523]; is a type of GO:0051051; is a type of negative regulation of multicellular organismal process [GO:0051241]; is a type of regulation of transcytosis [GO:1904298]; negatively regulates transcytosis [GO:0045056] Also known as: down regulation of transcytosis, down-regulation of transcytosis, downregulation of transcytosis, inhibition of transcytosis Definition: Any process that stops, prevents or reduces the frequency, rate or extent of transcytosis.